{
  "term_label": "very-low-density lipoprotein particle",
  "term_id": "GO:0034361",
  "gene_symbol": "APOC2",
  "gene": "UniProtKB:P02655",
  "gene_name": "Apolipoprotein C-II"
}